{
  "term_label": "chromatin",
  "gene_name": "Zinc finger protein 42 homolog",
  "gene_symbol": "ZFP42",
  "term_id": "GO:0000785",
  "gene": "UniProtKB:Q96MM3"
}